{
  "term_label": "SNARE complex assembly",
  "gene": "UniProtKB:P23763",
  "gene_name": "Vesicle-associated membrane protein 1",
  "gene_symbol": "VAMP1",
  "term_id": "GO:0035493"
}